negative regulation of branching morphogenesis of a nerve [GO:2000173] (biological process) Sources: GOC:BHF Definition: Any process that stops, prevents, or reduces the frequency, rate or extent of branching morphogenesis of a nerve. Relationships: is a type of negative regulation of developmental process [GO:0051093]; is a type of negative regulation of multicellular organismal process [GO:0051241]; is a type of GO:2000172; negatively regulates branching morphogenesis of a nerve [GO:0048755]